{
  "gene": "UniProtKB:Q9BRR9",
  "term_label": "small GTPase-mediated signal transduction",
  "gene_symbol": "ARHGAP9",
  "term_id": "GO:0007264",
  "gene_name": "Rho GTPase-activating protein 9"
}